{
  "gene_symbol": "DIP2A",
  "term_id": "UNKNOWN:0001",
  "term_label": "Unknown molecular function",
  "gene": "UniProtKB:Q14689",
  "gene_name": "Disco-interacting protein 2 homolog A"
}